pachytene [GO:0000239] (biological process) Note: Note that this term should not be used for direct annotation. If you are trying to make an annotation to x phase, it is likely that the correct annotation is 'regulation of x/y phase transition' or to a process which occurs during the reported phase (i.e mitotic DNA replication for mitotic S-phase). To capture the phase when a specific location or process is observed, the phase term can be used in an annotation extension (PMID:24885854) applied to a cellular component term (with the relation exists_during) or a biological process term (with the relation happens_during). Sources: GOC:mtg_cell_cycle Definition: The cell cycle phase which follows zygotene during prophase I of meiosis, and during which crossing over occurs between a chromatid in one partner and another chromatid in the homologous chromosome. Relationships: is a type of meiosis I cell cycle phase [GO:0098764]; is part of GO:0007128